sialyltransferase activity [GO:0008373] (molecular function) Relationships: is a type of glycosyltransferase activity [GO:0016757] Subtypes: GO:0001665, alpha-N-acetylneuraminate alpha-2,8-sialyltransferase activity [GO:0003828], beta-galactoside alpha-2,6-sialyltransferase activity [GO:0003835], beta-galactoside (CMP) alpha-2,3-sialyltransferase activity [GO:0003836], N-acetyllactosaminide alpha-2,3-sialyltransferase activity [GO:0008118], beta-D-galactosyl-(1->3)-N-acetyl-beta-D-galactosaminide alpha-2,3- sialyltransferase [GO:0047288], galactosyldiacylglycerol alpha-2,3-sialyltransferase activity [GO:0047289], alpha-N-acetylneuraminyl-2,3-beta-galactosyl-1,3-N-acetyl-galactosaminide 6-alpha-sialyltransferase activity [GO:0047290], GO:0047291, beta-galactoside alpha-2,3-sialyltransferase activity [GO:0052798] References: PMID:26192491 Sources: GOC:cjm Definition: Catalysis of the transfer of sialic acid to an acceptor molecule, typically the terminal portions of the sialylated glycolipids (gangliosides) or to the N- or O-linked sugar chains of glycoproteins.